{
  "term_label": "dendrite",
  "gene": "UniProtKB:Q96Q42",
  "term_id": "GO:0030425",
  "gene_name": "Alsin",
  "gene_symbol": "ALS2"
}